compound eye retinal cell programmed cell death [GO:0046667] (biological process) Relationships: is a type of retinal cell programmed cell death [GO:0046666]; is part of compound eye morphogenesis [GO:0001745] References: PMID:12006672 Definition: Programmed cell death that occurs in the retina to remove excess cells between ommatidia, thus resulting in a hexagonal lattice, precise with respect to cell number and position surrounding each ommatidium. Regulation: regulated by regulation of compound eye retinal cell programmed cell death [GO:0046669]; positively regulated by GO:0046672; negatively regulated by negative regulation of compound eye retinal cell programmed cell death [GO:0046673]